{
  "gene_symbol": "POLR2G",
  "gene_name": "DNA-directed RNA polymerase II subunit RPB7",
  "term_id": "GO:0000932",
  "term_label": "P-body",
  "gene": "UniProtKB:P62487"
}